hydrolase activity, hydrolyzing N-glycosyl compounds [GO:0016799] (molecular function) Subtypes: ADP-ribosylarginine hydrolase activity [GO:0003875], NAD+ nucleosidase activity [GO:0003953], purine nucleosidase activity [GO:0008477], AMP nucleosidase activity [GO:0008714], adenosylhomocysteine nucleosidase activity [GO:0008782], GO:0019104, NMN nucleosidase activity [GO:0019160], GO:0030597, GO:0033958, deoxyribodipyrimidine endonucleosidase activity [GO:0033959], GO:0033960, pyrimidine-5'-nucleotide nucleosidase activity [GO:0047405], GO:0047406, GO:0047407, GO:0047518, inosinate nucleosidase activity [GO:0047723], NADP+ nucleosidase activity [GO:0050135], ribosylpyrimidine nucleosidase activity [GO:0050263], NAD+ nucleosidase activity, cyclic ADP-ribose generating [GO:0061809], nicotinamide riboside hydrolase activity [GO:0070635], nicotinic acid riboside hydrolase activity [GO:0070636], GO:0070694, 6-amino-6-deoxyfutalosine hydrolase activity [GO:0102246], cytokinin riboside 5'-monophosphate phosphoribohydrolase activity [GO:0102682], ADP-ribosylserine hydrolase activity [GO:0140292], ADP-ribosylglutamate hydrolase activity [GO:0140293] Definition: Catalysis of the hydrolysis of any N-glycosyl bond. Sources: GOC:jl Relationships: is a type of GO:0016798